{
  "term_id": "UNKNOWN:0001",
  "term_label": "Unknown molecular function",
  "gene_name": "Uncharacterized protein C17orf113",
  "gene_symbol": "C17orf113",
  "gene": "UniProtKB:A0A1B0GUU1"
}